{
  "term_id": "GO:0005737",
  "term_label": "cytoplasm",
  "gene": "UniProtKB:Q9NWT6",
  "gene_symbol": "HIF1AN",
  "gene_name": "Hypoxia-inducible factor 1-alpha inhibitor"
}